{
  "term_id": "GO:0016485",
  "gene_name": "Transmembrane protease serine 13",
  "gene": "UniProtKB:Q9BYE2",
  "term_label": "protein processing",
  "gene_symbol": "TMPRSS13"
}